{
  "term_label": "immune response-inhibiting cell surface receptor signaling pathway",
  "gene": "UniProtKB:O76036",
  "term_id": "GO:0002767",
  "gene_symbol": "NCR1",
  "gene_name": "Natural cytotoxicity triggering receptor 1"
}